thymocyte migration [GO:0072679] (BP) Definition: The movement of a thymocyte through distinct intrathymic niches (e.g. medulla, cortex), where it receives a unique set of developmental cues required for T-cell development. Subtypes: extracellular matrix-dependent thymocyte migration [GO:0072680] Sources: CL:0000893, GOC:BHF, GOC:mah Also known as: thymic lymphocyte migration, immature T cell migration, immature T lymphocyte migration, immature T-cell migration, immature T-lymphocyte migration Regulation: regulated by regulation of thymocyte migration [GO:2000410]; negatively regulated by GO:2000411; positively regulated by positive regulation of thymocyte migration [GO:2000412] Relationships: is a type of T cell migration [GO:0072678]